{
  "gene_name": "UMP-CMP kinase 2, mitochondrial",
  "term_label": "dTMP kinase activity",
  "term_id": "GO:0004798",
  "gene": "UniProtKB:Q5EBM0",
  "gene_symbol": "CMPK2"
}